trans assembly of SL-containing precatalytic spliceosome [GO:0000352] (biological process) Sources: GOC:krc, GOC:mtg_mpo, ISBN:0879695897 Relationships: is a type of GO:0022618; is part of spliceosomal complex assembly [GO:0000245]; is part of GO:0045291 Also known as: trans assembly of spliced leader-containing precatalytic spliceosome Definition: Assembly of a spliceosomal complex containing the SL RNA and the pre-mRNA to be joined, as well as all the spliceosomal snRNPs involved in trans leader splicing. Formation of the trans leader spliceosome brings together the quadruple SL/U4/U5/U6 snRNP and the complex of the U2 snRNP with the splice site of the pre-mRNA.